{
  "gene": "UniProtKB:Q96EY8",
  "gene_name": "Corrinoid adenosyltransferase MMAB",
  "term_id": "GO:0008817",
  "gene_symbol": "MMAB",
  "term_label": "corrinoid adenosyltransferase activity"
}